{
  "term_label": "Unknown biological process",
  "gene_name": "Rabenosyn-5",
  "gene_symbol": "RBSN",
  "gene": "UniProtKB:Q9H1K0",
  "term_id": "UNKNOWN:0002"
}